hindgut contraction [GO:0043133] (biological process) Sources: GOC:jl, GOC:mtg_muscle, UBERON:0001046 Regulation: regulated by regulation of hindgut contraction [GO:0043134]; positively regulated by GO:0060450; negatively regulated by negative regulation of hindgut contraction [GO:0060451] Relationships: is a type of GO:0006939; is a type of digestive system process [GO:0022600] Definition: A process in which force is generated within smooth muscle tissue, resulting in a change in muscle geometry. This process occurs in the hindgut. Force generation involves a chemo-mechanical energy conversion step that is carried out by the actin/myosin complex activity, which generates force through ATP hydrolysis. The hindgut is the posterior part of the alimentary canal, including the rectum, and the large intestine.